{
  "gene_symbol": "ZNF154",
  "gene_name": "Zinc finger protein 154",
  "term_label": "regulation of transcription by RNA polymerase II",
  "term_id": "GO:0006357",
  "gene": "UniProtKB:Q13106"
}